positive regulation of endoplasmic reticulum unfolded protein response [GO:1900103] (biological process) Sources: GOC:TermGenie Also known as: activation of ER unfolded protein response, activation of erUPR, positive regulation of ER unfolded protein response, positive regulation of erUPR, up regulation of ER unfolded protein response, up regulation of endoplasmic reticulum unfolded protein response, up regulation of erUPR, up-regulation of ER unfolded protein response, up-regulation of endoplasmic reticulum unfolded protein response, up-regulation of erUPR, upregulation of ER unfolded protein response, upregulation of endoplasmic reticulum unfolded protein response, upregulation of erUPR, activation of endoplasmic reticulum unfolded protein response, activation of SREBP-mediated signalling pathway, positive regulation of SREBP-mediated signalling pathway, up regulation of SREBP-mediated signalling pathway, up-regulation of SREBP-mediated signalling pathway, upregulation of SREBP-mediated signalling pathway Definition: Any process that activates or increases the frequency, rate or extent of endoplasmic reticulum unfolded protein response. Subtypes: GO:1903893, GO:1903896, positive regulation of PERK-mediated unfolded protein response [GO:1903899] Relationships: is a type of regulation of endoplasmic reticulum unfolded protein response [GO:1900101]; is a type of positive regulation of intracellular signal transduction [GO:1902533]; is a type of GO:1905898; positively regulates endoplasmic reticulum unfolded protein response [GO:0030968]